{
  "term_id": "GO:0005164",
  "gene_symbol": "TRIM37",
  "gene_name": "E3 ubiquitin-protein ligase TRIM37",
  "term_label": "tumor necrosis factor receptor binding",
  "gene": "UniProtKB:O94972"
}